{
  "gene_symbol": "SIRPB2",
  "term_id": "UNKNOWN:0002",
  "gene": "UniProtKB:Q5JXA9",
  "gene_name": "Signal-regulatory protein beta-2",
  "term_label": "Unknown biological process"
}